{
  "gene_name": "Carboxypeptidase A5",
  "gene": "UniProtKB:Q8WXQ8",
  "term_id": "GO:0006508",
  "gene_symbol": "CPA5",
  "term_label": "proteolysis"
}